histone H3K4 methyltransferase activity [GO:0042800] (molecular function) Also known as: histone H3 lysine 4-specific methyltransferase activity, histone H3K4 methylase activity, histone lysine N-methyltransferase activity (H3-K4 specific), histone methylase activity (H3-K4 specific), histone methyltransferase activity (H3-K4 specific), histone-H3K4 methyltransferase activity Note: Comment: Note that the residue position corresponds to the canonical human H3 histone (UniProtKB:P84243); this residue is conserved across all eukaryotes. Residue 1 is the first residue following removal of the initiating Methionine (Met). Note that each histone is encoded by multiple genes, and sequences may vary across different genes within an organism. Relationships: is a type of protein-lysine N-methyltransferase activity [GO:0016279]; is a type of histone H3 methyltransferase activity [GO:0140938] Definition: Catalysis of the reaction: S-adenosyl-L-methionine + histone H3 L-lysine (position 4) = S-adenosyl-L-homocysteine + histone H3 N6-methyl-L-lysine (position 4). This reaction is the addition of up to three methyl groups to the lysine residue at position 4 of the histone H3 protein. References: PMID:12086618 Subtypes: GO:0140945, GO:0140946, histone H3K4 trimethyltransferase activity [GO:0140999]